positive regulation of microtubule polymerization [GO:0031116] (biological process) Also known as: up regulation of microtubule polymerization, up-regulation of microtubule polymerization, upregulation of microtubule polymerization, activation of microtubule polymerization, stimulation of microtubule polymerization Sources: GOC:mah Relationships: is a type of positive regulation of microtubule polymerization or depolymerization [GO:0031112]; is_a regulation of microtubule polymerization [GO:0031113]; is a type of positive regulation of protein polymerization [GO:0032273]; is a type of positive regulation of supramolecular fiber organization [GO:1902905]; positively regulates microtubule polymerization [GO:0046785] Definition: Any process that activates or increases the frequency, rate or extent of microtubule polymerization. Subtypes: GO:0090063